{
  "gene": "UniProtKB:Q9BRG1",
  "gene_name": "Vacuolar protein-sorting-associated protein 25",
  "term_id": "GO:0005198",
  "term_label": "structural molecule activity",
  "gene_symbol": "VPS25"
}